excitatory neuromuscular junction [GO:0098520] (CC) Sources: GOC:dos Relationships: is_a neuromuscular junction [GO:0031594]; is a type of excitatory synapse [GO:0060076] Definition: The junction between the axon of a motor neuron and a muscle fiber. In response to the arrival of action potentials, the presynaptic button releases molecules of neurotransmitters into the synaptic cleft. These diffuse across the cleft and transmit the signal to the postsynaptic membrane of the muscle fiber, leading to a post-synaptic potential responsible for muscle contraction. Subtypes: neuromuscular junction of skeletal muscle fiber [GO:0098522], GO:0098525